{
  "gene": "UniProtKB:P50851",
  "term_label": "protein localization to phagophore assembly site",
  "gene_name": "Lipopolysaccharide-responsive and beige-like anchor protein",
  "term_id": "GO:0034497",
  "gene_symbol": "LRBA"
}